{
  "term_id": "GO:0031462",
  "term_label": "Cul2-RING ubiquitin ligase complex",
  "gene": "UniProtKB:Q9HCJ5",
  "gene_symbol": "ZSWIM6",
  "gene_name": "Zinc finger SWIM domain-containing protein 6"
}